{
  "gene": "UniProtKB:O95868",
  "gene_symbol": "LY6G6D",
  "term_id": "GO:0030550",
  "term_label": "acetylcholine receptor inhibitor activity",
  "gene_name": "Lymphocyte antigen 6 complex locus protein G6d"
}